{
  "gene": "UniProtKB:Q16531",
  "term_id": "GO:0005634",
  "gene_symbol": "DDB1",
  "term_label": "nucleus",
  "gene_name": "DNA damage-binding protein 1"
}